{
  "gene": "UniProtKB:P62877",
  "term_label": "nucleus",
  "term_id": "GO:0005634",
  "gene_symbol": "RBX1",
  "gene_name": "E3 ubiquitin-protein ligase RBX1"
}